gerfelin catabolic process [GO:1900577] (BP) Also known as: gerfelin breakdown, gerfelin catabolism, gerfelin degradation Definition: The chemical reactions and pathways resulting in the breakdown of gerfelin. Sources: GOC:TermGenie, GOC:di Relationships: is a type of catechol-containing compound catabolic process [GO:0019614]; is a type of benzene-containing compound metabolic process [GO:0042537]; is a type of carboxylic acid catabolic process [GO:0046395]; is a type of GO:0090487; is a type of ether catabolic process [GO:1901502]